{
  "gene_symbol": "ABHD2",
  "gene": "UniProtKB:P08910",
  "term_id": "GO:0051792",
  "gene_name": "Monoacylglycerol lipase ABHD2",
  "term_label": "medium-chain fatty acid biosynthetic process"
}